{
  "gene_name": "MOB kinase activator 3B",
  "gene": "UniProtKB:Q86TA1",
  "gene_symbol": "MOB3B",
  "term_id": "GO:0005737",
  "term_label": "cytoplasm"
}